{
  "gene_symbol": "SLCO2A1",
  "term_id": "GO:0015732",
  "term_label": "prostaglandin transport",
  "gene_name": "Solute carrier organic anion transporter family member 2A1",
  "gene": "UniProtKB:Q92959"
}